{
  "gene_name": "Natriuretic peptides A",
  "term_id": "GO:0003085",
  "term_label": "negative regulation of systemic arterial blood pressure",
  "gene": "UniProtKB:P01160",
  "gene_symbol": "NPPA"
}